positive regulation of mitotic DNA damage checkpoint [GO:1904291] (biological process) Definition: Any process that activates or increases the frequency, rate or extent of mitotic DNA damage checkpoint. Also known as: up regulation of mitotic DNA damage checkpoint, up-regulation of mitotic DNA damage checkpoint, upregulation of mitotic DNA damage checkpoint, activation of mitotic DNA damage checkpoint References: PMID:16549501 Sources: GOC:TermGenie, GOC:kmv, GO_REF:0000058 Relationships: is_a positive regulation of cell cycle process [GO:0090068]; is a type of regulation of mitotic DNA damage checkpoint [GO:1904289]; is a type of GO:2000003; positively regulates GO:0044773